{
  "gene_symbol": "NLK",
  "term_label": "intracellular signal transduction",
  "gene": "UniProtKB:Q9UBE8",
  "term_id": "GO:0035556",
  "gene_name": "Serine_threonine-protein kinase NLK"
}